2-polyprenylphenol 6-hydroxylase activity [GO:0019168] (molecular function) Sources: RHEA:55892 Also known as: 2-octaprenylphenol hydroxylase activity Definition: Catalysis of the reaction: a 2-(all-trans-polyprenyl)phenol + NADPH + O2 + H+ = a 3-(all-trans-polyprenyl)benzene-1,2-diol + NADP+ + H2O. Relationships: is a type of oxidoreductase activity, acting on paired donors, with incorporation or reduction of molecular oxygen, NAD(P)H as one donor, and incorporation of one atom of oxygen [GO:0016709]